elongation of arista core [GO:0035015] (biological process) References: PMID:11404081 Sources: GOC:bf Definition: The increase in length of the aristal core. The arista is the terminal segment of the antenna and consists of a central core and a series of lateral extensions. Relationships: is a type of developmental growth involved in morphogenesis [GO:0060560]; is part of antennal morphogenesis [GO:0048800]